{
  "term_id": "GO:0007411",
  "term_label": "axon guidance",
  "gene": "UniProtKB:O94856",
  "gene_symbol": "NFASC",
  "gene_name": "Neurofascin"
}